{
  "term_label": "regulation of DNA damage checkpoint",
  "gene_symbol": "WDR76",
  "term_id": "GO:2000001",
  "gene": "UniProtKB:Q9H967",
  "gene_name": "WD repeat-containing protein 76"
}